{
  "gene": "UniProtKB:A0PJX4",
  "term_label": "Unknown cellular component",
  "gene_name": "Protein shisa-3 homolog",
  "term_id": "UNKNOWN:0003",
  "gene_symbol": "SHISA3"
}